{
  "gene_symbol": "Q1T7F1",
  "term_id": "UNKNOWN:0003",
  "gene_name": "Putative chemokine-related protein B42",
  "gene": "UniProtKB:Q1T7F1",
  "term_label": "Unknown cellular component"
}